{
  "gene": "UniProtKB:Q16394",
  "term_label": "Golgi apparatus",
  "gene_symbol": "EXT1",
  "term_id": "GO:0005794",
  "gene_name": "Exostosin-1"
}